secondary active sulfate transmembrane transporter activity [GO:0008271] (MF) Relationships: is a type of GO:0015116; is a type of GO:0015291 Subtypes: sulfate:proton symporter activity [GO:0008512], high-affinity sulfate transmembrane transporter activity [GO:0015381], sodium:sulfate symporter activity [GO:0015382], GO:0015383, GO:0160044 Also known as: secondary active sulphate transmembrane transporter activity, sulphate porter activity, sulfate porter activity Sources: GOC:mtg_transport Definition: Enables the secondary active transfer of sulfate from one side of a membrane to the other. Secondary active transport is the transfer of a solute across a membrane, up its concentration gradient. The transporter binds the solute and undergoes a series of conformational changes. Transport works equally well in either direction and is driven by a chemiosmotic source of energy. Secondary active transporters include symporters and antiporters.